{
  "gene_name": "ER membrane protein complex subunit 9",
  "gene_symbol": "EMC9",
  "term_label": "membrane insertase activity",
  "term_id": "GO:0032977",
  "gene": "UniProtKB:Q9Y3B6"
}